{
  "gene_symbol": "NOS3",
  "term_id": "GO:0010181",
  "gene": "UniProtKB:P29474",
  "term_label": "FMN binding",
  "gene_name": "Nitric oxide synthase 3"
}